{
  "gene": "UniProtKB:Q13873",
  "term_id": "GO:0005024",
  "gene_symbol": "BMPR2",
  "term_label": "transforming growth factor beta receptor activity",
  "gene_name": "Bone morphogenetic protein receptor type-2"
}